{
  "term_id": "GO:0000902",
  "gene": "UniProtKB:P40123",
  "term_label": "cell morphogenesis",
  "gene_name": "Adenylyl cyclase-associated protein 2",
  "gene_symbol": "CAP2"
}